iron-iron nitrogenase complex [GO:0016611] (cellular component) Relationships: is a type of nitrogenase complex [GO:0016610] References: PMID:11848850 Sources: GOC:jl Note: Note that it is not established whether the nitrogenase exists in vivo in a specific particle or whether the nitrogenase proteins are bound nonspecifically to the membranes of some cells. Definition: An enzyme complex containing an iron-iron cluster found in species such as the photosynthetic bacterium Rhodobacter capsulatus. It is composed of two main subunits, dinitrogenase and nitrogenase reductase. Dinitrogenase, the iron-iron containing subunit, has an alpha1-beta2 or alpha2-beta2 structure, and the nitrogenase reductase subunit is a homodimer. Functions in the catalysis of the formation of oxidized ferredoxin and ammonia from reduced ferredoxin and nitrogen.